{
  "gene_symbol": "CIB2",
  "gene_name": "Calcium and integrin-binding family member 2",
  "term_id": "GO:0071944",
  "term_label": "cell periphery",
  "gene": "UniProtKB:O75838"
}